{
  "term_id": "GO:0000422",
  "gene_name": "Ubiquitin-like protein ATG12",
  "term_label": "autophagy of mitochondrion",
  "gene_symbol": "ATG12",
  "gene": "UniProtKB:O94817"
}